{
  "gene": "UniProtKB:Q15286",
  "term_id": "GO:0003924",
  "gene_symbol": "RAB35",
  "gene_name": "Ras-related protein Rab-35",
  "term_label": "GTPase activity"
}